{
  "gene_symbol": "PLXNA3",
  "term_id": "GO:0002116",
  "gene_name": "Plexin-A3",
  "term_label": "semaphorin receptor complex",
  "gene": "UniProtKB:P51805"
}